{
  "gene_symbol": "FGF9",
  "gene": "UniProtKB:P31371",
  "gene_name": "Fibroblast growth factor 9",
  "term_label": "growth factor activity",
  "term_id": "GO:0008083"
}